{
  "term_id": "GO:0005886",
  "gene": "UniProtKB:Q9HCH3",
  "term_label": "plasma membrane",
  "gene_name": "Copine-5",
  "gene_symbol": "CPNE5"
}